gluconate transmembrane transporter activity [GO:0015128] (molecular function) Relationships: is a type of aldonate transmembrane transporter activity [GO:0042879]; is part of gluconate transmembrane transport [GO:0035429] Definition: Enables the transfer of gluconate from one side of a membrane to the other. Gluconate is the aldonic acid derived from glucose. Sources: GOC:ai, ISBN:0198506732 Also known as: L-idonate/D-gluconate:hydrogen symporter activity